{
  "term_id": "UNKNOWN:0001",
  "gene": "UniProtKB:Q6UXV4",
  "gene_name": "MICOS complex subunit MIC27",
  "gene_symbol": "APOOL",
  "term_label": "Unknown molecular function"
}